{
  "term_label": "Unknown molecular function",
  "gene_name": "BLOC-2 complex member HPS3",
  "term_id": "UNKNOWN:0001",
  "gene_symbol": "HPS3",
  "gene": "UniProtKB:Q969F9"
}